{
  "term_id": "GO:0032777",
  "gene_name": "Enhancer of polycomb homolog 2",
  "term_label": "piccolo histone acetyltransferase complex",
  "gene": "UniProtKB:Q52LR7",
  "gene_symbol": "EPC2"
}